{
  "term_id": "GO:0007265",
  "term_label": "Ras protein signal transduction",
  "gene": "UniProtKB:Q07890",
  "gene_name": "Son of sevenless homolog 2",
  "gene_symbol": "SOS2"
}